{
  "term_label": "Wnt receptor activity",
  "gene_symbol": "FZD2",
  "gene_name": "Frizzled-2",
  "gene": "UniProtKB:Q14332",
  "term_id": "GO:0042813"
}